{
  "term_id": "UNKNOWN:0002",
  "gene_name": "TATA element modulatory factor",
  "gene_symbol": "TMF1",
  "gene": "UniProtKB:P82094",
  "term_label": "Unknown biological process"
}